regulation of isotype switching to IgA isotypes [GO:0048296] (biological process) Also known as: regulation of class switch recombination to IgA isotypes, regulation of class switching to IgA isotypes, regulation of isotype switch recombination to IgA isotypes Relationships: is a type of regulation of isotype switching [GO:0045191]; regulates isotype switching to IgA isotypes [GO:0048290] Definition: Any process that modulates the frequency, rate or extent of isotype switching to IgA isotypes. Sources: GOC:jid Subtypes: negative regulation of isotype switching to IgA isotypes [GO:0048297], positive regulation of isotype switching to IgA isotypes [GO:0048298]